maintenance of shoot apical meristem identity [GO:0010492] (biological process) Definition: The process in which an organism retains a population of shoot apical meristem cells, preventing the commitment of all stem cell progeny to a differentiated cell fate. References: PMID:17461786 Sources: GOC:dph, GOC:tb Relationships: is a type of maintenance of meristem identity [GO:0010074]